{
  "term_label": "postsynaptic membrane",
  "term_id": "GO:0045211",
  "gene": "UniProtKB:Q9UPX8",
  "gene_name": "SH3 and multiple ankyrin repeat domains protein 2",
  "gene_symbol": "SHANK2"
}